positive regulation of triglyceride metabolic process [GO:0090208] (biological process) Subtypes: positive regulation of triglyceride biosynthetic process [GO:0010867], positive regulation of triglyceride catabolic process [GO:0010898] Definition: Any process that increases the frequency, rate or extent of the chemical reactions and pathways involving triglyceride, any triester of glycerol. Sources: GOC:dph, GOC:sl, GOC:tb Relationships: is a type of GO:0045834; is a type of regulation of triglyceride metabolic process [GO:0090207]; positively regulates triglyceride metabolic process [GO:0006641]